{
  "gene_name": "Olfactory receptor 5AS1",
  "gene": "UniProtKB:Q8N127",
  "term_id": "UNKNOWN:0002",
  "term_label": "Unknown biological process",
  "gene_symbol": "OR5AS1"
}